RNA polymerase II cis-regulatory region sequence-specific DNA binding [GO:0000978] (molecular function) Relationships: is a type of RNA polymerase II transcription regulatory region sequence-specific DNA binding [GO:0000977]; is a type of GO:0000987 Sources: GOC:txnOH-2018 Subtypes: serum response element binding [GO:0010736], sterol response element binding [GO:0032810], GO:0034056, GO:0035497, carbohydrate response element binding [GO:0035538], retinoic acid-responsive element binding [GO:0044323], GO:0044377, juvenile hormone response element binding [GO:0070594], vitamin D response element binding [GO:0070644], GO:0070888, GO:0071820, GC-box binding [GO:0140728] Definition: Binding to a specific upstream regulatory DNA sequence (transcription factor recognition sequence or binding site) located in cis relative to the transcription start site (i.e., on the same strand of DNA) of a gene transcribed by RNA polymerase II. Note: Note that the phrase "upstream activating sequence", or UAS is often used in S. cerevisiae literature to refer to cis-regulatory sequences. In bacteria such as E. coli, the phrase "upstream activating sequence", or UAS is usually a synonym for "enhancer". Also known as: RNA polymerase II core promoter proximal region sequence-specific DNA binding, RNA polymerase II distal enhancer sequence-specific DNA binding, RNA polymerase II promoter proximal region sequence-specific DNA binding, RNA polymerase II proximal promoter sequence-specific DNA binding, RNA polymerase II upstream activating sequence (UAS) sequence-specific DNA binding